{
  "gene": "UniProtKB:C9JC47",
  "gene_symbol": "FAM157A",
  "term_id": "UNKNOWN:0002",
  "term_label": "Unknown biological process",
  "gene_name": "Putative protein FAM157A"
}